{
  "gene_symbol": "MAP3K13",
  "term_id": "GO:0005737",
  "term_label": "cytoplasm",
  "gene_name": "Mitogen-activated protein kinase kinase kinase 13",
  "gene": "UniProtKB:O43283"
}